{
  "term_id": "GO:0007507",
  "gene_symbol": "PDLIM4",
  "gene_name": "PDZ and LIM domain protein 4",
  "term_label": "heart development",
  "gene": "UniProtKB:P50479"
}